succinate-semialdehyde dehydrogenase binding [GO:0032145] (molecular function) Also known as: succinic semialdehyde dehydrogenase binding Sources: GOC:mah Definition: Binding to succinate-semialdehyde dehydrogenase. Relationships: is a type of enzyme binding [GO:0019899]